negative regulation of fibroblast migration [GO:0010764] (biological process) Definition: Any process that decreases the rate, frequency or extent of fibroblast cell migration. Fibroblast cell migration is accomplished by extension and retraction of a pseudopodium. Subtypes: negative regulation of hepatic stellate cell migration [GO:0061871] Sources: GOC:dph, GOC:tb Relationships: is a type of regulation of fibroblast migration [GO:0010762]; is a type of negative regulation of cell migration [GO:0030336]; negatively regulates fibroblast migration [GO:0010761] Also known as: negative regulation of fibroblast cell migration